{
  "term_label": "DNA-binding transcription factor activity, RNA polymerase II-specific",
  "gene": "UniProtKB:P84022",
  "gene_symbol": "SMAD3",
  "term_id": "GO:0000981",
  "gene_name": "Mothers against decapentaplegic homolog 3"
}